{
  "term_id": "UNKNOWN:0003",
  "term_label": "Unknown cellular component",
  "gene_name": "Putative uncharacterized protein C1orf140",
  "gene": "UniProtKB:Q5VVS0",
  "gene_symbol": "C1orf140"
}